positive regulation of mitochondrial DNA metabolic process [GO:1901860] (biological process) Definition: Any process that activates or increases the frequency, rate or extent of mitochondrial DNA metabolic process. Also known as: activation of mitochondrial DNA metabolism, activation of mtDNA metabolic process, activation of mtDNA metabolism, positive regulation of mitochondrial DNA metabolism, positive regulation of mtDNA metabolic process, positive regulation of mtDNA metabolism, up regulation of mitochondrial DNA metabolic process, up regulation of mitochondrial DNA metabolism, up regulation of mtDNA metabolic process, up regulation of mtDNA metabolism, up-regulation of mitochondrial DNA metabolic process, up-regulation of mitochondrial DNA metabolism, up-regulation of mtDNA metabolic process, up-regulation of mtDNA metabolism, upregulation of mitochondrial DNA metabolic process, upregulation of mitochondrial DNA metabolism, upregulation of mtDNA metabolic process, upregulation of mtDNA metabolism, activation of mitochondrial DNA metabolic process References: PMID:23150719 Sources: GOC:TermGenie, GOC:yaf Subtypes: GO:0090297 Relationships: is a type of positive regulation of organelle organization [GO:0010638]; is a type of regulation of mitochondrion organization [GO:0010821]; is a type of positive regulation of DNA metabolic process [GO:0051054]; is a type of GO:1901858; positively regulates mitochondrion organization [GO:0007005]; positively regulates mitochondrial DNA metabolic process [GO:0032042]